regulation of proteolysis [GO:0030162] (biological process) Relationships: is a type of regulation of protein metabolic process [GO:0051246]; regulates proteolysis [GO:0006508] Sources: GOC:mah Also known as: regulation of peptidolysis Subtypes: negative regulation of proteolysis [GO:0045861], positive regulation of proteolysis [GO:0045862], regulation of membrane protein ectodomain proteolysis [GO:0051043], regulation of peptidase activity [GO:0052547], GO:0070613, GO:1903050 Definition: Any process that modulates the frequency, rate or extent of the hydrolysis of a peptide bond or bonds within a protein.